axial mesoderm development [GO:0048318] (biological process) Relationships: is_a mesoderm development [GO:0007498] Sources: GOC:dgh Definition: The process whose specific outcome is the progression of the axial mesoderm over time, from its formation to the mature structure. The axial mesoderm includes the prechordal mesoderm and the chordamesoderm. It gives rise to the prechordal plate and to the notochord.